{
  "gene_symbol": "RAB6B",
  "gene_name": "Ras-related protein Rab-6B",
  "gene": "UniProtKB:Q9NRW1",
  "term_label": "intracellular protein transport",
  "term_id": "GO:0006886"
}